10-formyltetrahydrofolate metabolic process [GO:0009256] (biological process) Sources: GOC:ai Relationships: is a type of dicarboxylic acid metabolic process [GO:0043648]; is a type of tetrahydrofolate metabolic process [GO:0046653] Subtypes: 10-formyltetrahydrofolate biosynthetic process [GO:0009257], 10-formyltetrahydrofolate catabolic process [GO:0009258] Definition: The chemical reactions and pathways involving 10-formyltetrahydrofolate, the formylated derivative of tetrahydrofolate. Also known as: 10-formyl-THF metabolic process, 10-formyl-THF metabolism, 10-formyltetrahydrofolate metabolism